{
  "gene_symbol": "SEPTIN9",
  "gene_name": "Septin-9",
  "term_label": "cell division site",
  "term_id": "GO:0032153",
  "gene": "UniProtKB:Q9UHD8"
}